egg chorion [GO:0042600] (cellular component) Sources: GOC:jl, ISBN:0721662544 Note: Note that this term does not refer to the extraembryonic membrane surrounding the embryo of amniote vertebrates as this is an anatomical structure and is therefore not covered by GO. Relationships: is a type of external encapsulating structure [GO:0030312] Definition: A protective, noncellular membrane that surrounds the eggs of various animals including insects and fish.